{
  "gene_symbol": "FOXD4L6",
  "gene_name": "Forkhead box protein D4-like 6",
  "term_label": "anatomical structure morphogenesis",
  "term_id": "GO:0009653",
  "gene": "UniProtKB:Q3SYB3"
}